mediolateral intercalation [GO:0060031] (BP) Relationships: is a type of cell migration involved in gastrulation [GO:0042074]; is part of convergent extension involved in gastrulation [GO:0060027] Definition: The interdigitation of cells along the mediolateral axis during gastrulation. References: PMID:12062082 Sources: GOC:dgf, GOC:dph